{
  "gene": "UniProtKB:Q12967",
  "term_label": "guanyl-nucleotide exchange factor activity",
  "term_id": "GO:0005085",
  "gene_symbol": "RALGDS",
  "gene_name": "Ral guanine nucleotide dissociation stimulator"
}